{
  "term_label": "endocytic recycling",
  "gene": "UniProtKB:Q8N1B4",
  "gene_symbol": "VPS52",
  "term_id": "GO:0032456",
  "gene_name": "Vacuolar protein sorting-associated protein 52 homolog"
}